{
  "gene": "UniProtKB:Q9GZN2",
  "term_label": "RNA polymerase II cis-regulatory region sequence-specific DNA binding",
  "gene_symbol": "TGIF2",
  "term_id": "GO:0000978",
  "gene_name": "Homeobox protein TGIF2"
}